regulation of glycolytic fermentation to ethanol [GO:2001154] (biological process) Subtypes: GO:2001155, positive regulation of glycolytic fermentation to ethanol [GO:2001172] Also known as: regulation of ethanol fermentation, regulation of glucose fermentation to ethanol Definition: Any process that modulates the frequency, rate or extent of glucose catabolic process to ethanol. Relationships: is a type of GO:0043470; is a type of GO:0062012; regulates pyruvate fermentation to ethanol [GO:0019655] Sources: GOC:obol